{
  "gene": "UniProtKB:Q5K130",
  "term_id": "UNKNOWN:0002",
  "gene_symbol": "CLLU1-AS1",
  "gene_name": "Putative uncharacterized protein CLLU1-AS1",
  "term_label": "Unknown biological process"
}